regulation of systemic arterial blood pressure by hormone [GO:0001990] (biological process) Definition: The process in which hormones modulate the force with which blood passes through the circulatory system. A hormone is one of a group of substances formed in very small amounts in one specialized organ or group of cells and carried (sometimes in the bloodstream) to another organ or group of cells, in the same organism, upon which they have a specific regulatory action. Relationships: is a type of regulation of systemic arterial blood pressure mediated by a chemical signal [GO:0003044]; is a type of endocrine process [GO:0050886] Subtypes: regulation of systemic arterial blood pressure by vasopressin [GO:0001992], GO:0002017, GO:0003050, GO:0003067, GO:0003081, regulation of systemic arterial blood pressure by endothelin [GO:0003100], regulation of systemic arterial blood pressure by circulatory epinephrine-norepinephrine [GO:0003101] Also known as: blood pressure regulation by hormone, hormonal regulation of blood pressure, hormonal control of blood pressure Sources: GOC:mtg_cardio, ISBN:0721643949